transcriptional attenuation [GO:0031555] (biological process) References: PMID:12210530, PMID:15851059, PMID:7007895 Relationships: is a type of negative regulation of gene expression [GO:0010629]; is a type of positive regulation of termination of DNA-templated transcription [GO:0060566] Subtypes: transcriptional attenuation by ribosome [GO:0031556] Definition: A negative regulation of gene expression mechanism by which bacteria and archae can direct RNA polymerase to prematurely terminate transcription in response to a specific metabolic signal.